{
  "gene_name": "Centrosomal protein of 104 kDa",
  "term_label": "cilium",
  "gene_symbol": "CEP104",
  "term_id": "GO:0005929",
  "gene": "UniProtKB:O60308"
}